{
  "term_label": "Unknown molecular function",
  "gene_name": "Late cornified envelope protein 2D",
  "gene_symbol": "LCE2D",
  "gene": "UniProtKB:Q5TA82",
  "term_id": "UNKNOWN:0001"
}